clathrin-coated vesicle cargo loading, AP-1-mediated [GO:0035653] (biological process) References: PMID:12802059, PMID:16162817 Sources: GOC:lb Definition: Formation of a macromolecular complex between proteins of the AP-1 adaptor complex and proteins and/or lipoproteins that are going to be transported by a clathrin-coated vesicle. The AP-1 adaptor protein complex is a component of the cytoplasmic coat found on clathrin-coated vesicles, and binds to sorting signals of cargo to facilitate their trafficking. Relationships: is a type of clathrin-coated vesicle cargo loading [GO:0035652] Also known as: cargo loading into clathrin-coated vesicle, AP-1-mediated